{
  "term_id": "GO:0005886",
  "term_label": "plasma membrane",
  "gene_symbol": "PLPP3",
  "gene_name": "Phospholipid phosphatase 3",
  "gene": "UniProtKB:O14495"
}